purine nucleotide catabolic process [GO:0006195] (biological process) Regulation: regulated by regulation of purine nucleotide catabolic process [GO:0033121]; negatively regulated by negative regulation of purine nucleotide catabolic process [GO:0033122]; positively regulated by positive regulation of purine nucleotide catabolic process [GO:0033123] Sources: GOC:go_curators, ISBN:0198506732 Subtypes: NADP+ catabolic process [GO:0006742], purine ribonucleotide catabolic process [GO:0009154], purine deoxyribonucleotide catabolic process [GO:0009155], NAD+ catabolic process [GO:0019677] Definition: The chemical reactions and pathways resulting in the breakdown of a purine nucleotide, a compound consisting of nucleoside (a purine base linked to a deoxyribose or ribose sugar) esterified with a phosphate group at either the 3' or 5'-hydroxyl group of the sugar. Relationships: is a type of purine nucleotide metabolic process [GO:0006163]; is a type of nucleotide catabolic process [GO:0009166]; is_a GO:0072523 Also known as: purine nucleotide breakdown, purine nucleotide catabolism, purine nucleotide degradation